peptidoglycan transmembrane transporter activity [GO:0015647] (molecular function) Also known as: murein transporter activity Sources: GOC:ai Subtypes: peptidoglycan peptide transmembrane transporter activity [GO:0015640], lipid-linked peptidoglycan transporter activity [GO:0015648] Definition: Enables the transfer of peptidoglycans, a class of glycoconjugates found in bacterial cell walls, from one side of a membrane to the other. Relationships: is a type of macromolecule transmembrane transporter activity [GO:0022884]; is a type of carbohydrate derivative transmembrane transporter activity [GO:1901505]; is part of peptidoglycan transport [GO:0015835]